{
  "gene_name": "ER membrane protein complex subunit 10",
  "term_label": "Unknown molecular function",
  "gene": "UniProtKB:Q5UCC4",
  "term_id": "UNKNOWN:0001",
  "gene_symbol": "EMC10"
}